positive regulation of podocyte apoptotic process [GO:1904635] (biological process) Also known as: positive regulation of glomerular podocyte apoptotic process, positive regulation of glomerular visceral epithelial cell apoptotic process, up regulation of glomerular podocyte apoptotic process, up regulation of glomerular visceral epithelial cell apoptotic process, up regulation of podocyte apoptotic process, up-regulation of glomerular podocyte apoptotic process, up-regulation of glomerular visceral epithelial cell apoptotic process, up-regulation of podocyte apoptotic process, upregulation of glomerular podocyte apoptotic process, upregulation of glomerular visceral epithelial cell apoptotic process, upregulation of podocyte apoptotic process, activation of glomerular podocyte apoptosis, activation of glomerular podocyte apoptotic process, activation of glomerular visceral epithelial cell apoptosis, activation of glomerular visceral epithelial cell apoptotic process, activation of podocyte apoptosis, activation of podocyte apoptotic process, positive regulation of glomerular podocyte apoptosis, positive regulation of glomerular visceral epithelial cell apoptosis, positive regulation of podocyte apoptosis, up regulation of glomerular podocyte apoptosis, up regulation of glomerular visceral epithelial cell apoptosis, up regulation of podocyte apoptosis, up-regulation of glomerular podocyte apoptosis, up-regulation of glomerular visceral epithelial cell apoptosis, up-regulation of podocyte apoptosis, upregulation of glomerular podocyte apoptosis, upregulation of glomerular visceral epithelial cell apoptosis, upregulation of podocyte apoptosis Relationships: is a type of positive regulation of epithelial cell apoptotic process [GO:1904037]; is a type of regulation of podocyte apoptotic process [GO:1904633]; positively regulates podocyte apoptotic process [GO:1903210] References: PMID:23692924 Sources: GOC:TermGenie, GO_REF:0000058 Definition: Any process that activates or increases the frequency, rate or extent of glomerular visceral epithelial cell apoptotic process.